{
  "term_label": "Unknown biological process",
  "gene_name": "Tubulin epsilon and delta complex protein 2",
  "term_id": "UNKNOWN:0002",
  "gene": "UniProtKB:Q7L2K0",
  "gene_symbol": "TEDC2"
}